{
  "term_label": "calcium-dependent protein serine/threonine phosphatase regulator activity",
  "gene_symbol": "RCAN1",
  "term_id": "GO:0008597",
  "gene": "UniProtKB:P53805",
  "gene_name": "Calcipressin-1"
}